{
  "term_label": "Unknown cellular component",
  "gene": "UniProtKB:Q7RTZ1",
  "gene_symbol": "OVCH2",
  "gene_name": "Ovochymase-2",
  "term_id": "UNKNOWN:0003"
}